ecdysteroid UDP-glucosyltransferase activity [GO:0050488] (molecular function) Relationships: is a type of GO:0035251 References: PMID:10073711 Sources: GOC:ai Also known as: ecdysteroid UDP-glucosyl/UDP-glucuronosyl transferase activity Definition: Catalysis of the reaction: UDP-glucose + ecdysteroid = UDP + glucosyl-ecdysteroid.